{
  "gene": "UniProtKB:Q8NDA8",
  "gene_name": "Maestro heat-like repeat-containing protein family member 1",
  "term_id": "GO:0005737",
  "gene_symbol": "MROH1",
  "term_label": "cytoplasm"
}